ATPase coupled ion transmembrane transporter activity involved in regulation of presynaptic membrane potential [GO:0099521] (molecular function) Definition: Any ATPase coupled ion transmembrane transporter activity, occurring in the presynaptic membrane, that is involved in regulation of presynaptic membrane potential. References: PMID:17220883 Sources: GOC:dos Also known as: ATPase coupled ion transmembrane transporter activity involved in regulation of pre-synaptic membrane potential, ATPase-coupled ion transmembrane transporter activity involved in regulation of presynaptic membrane potential Relationships: is a type of GO:0042625; BFO_0000050 regulation of presynaptic membrane potential [GO:0099505]; occurs in GO:0042734